{
  "gene": "UniProtKB:Q8N0X2",
  "gene_symbol": "SPAG16",
  "term_label": "axoneme assembly",
  "term_id": "GO:0035082",
  "gene_name": "Sperm-associated antigen 16 protein"
}